{
  "term_id": "GO:0050911",
  "gene": "UniProtKB:Q8NGW6",
  "gene_symbol": "OR6K6",
  "gene_name": "Olfactory receptor 6K6",
  "term_label": "detection of chemical stimulus involved in sensory perception of smell"
}